cellular response to dodecane [GO:1902787] (BP) Relationships: is a type of cellular response to alkane [GO:1902779]; is a type of response to dodecane [GO:1902786] Definition: Any process that results in a change in state or activity of a cell (in terms of movement, secretion, enzyme production, gene expression, etc.) as a result of a dodecane stimulus. References: PMID:23826995 Sources: GOC:TermGenie, GOC:mengo_curators, GO_REF:0000071